{
  "gene_symbol": "FGFR1",
  "gene_name": "Fibroblast growth factor receptor 1",
  "term_id": "GO:0043235",
  "gene": "UniProtKB:P11362",
  "term_label": "receptor complex"
}